tRNA N(6)-L-threonylcarbamoyladenine synthase activity [GO:0061711] (molecular function) Also known as: N(6)-L-threonylcarbamoyladenine synthase activity, t6A synthase activity Definition: Catalysis of the reaction: L-threonylcarbamoyladenylate + adenine(37) in tRNA = AMP + N(6)-L-threonylcarbamoyladenine(37) in tRNA. Relationships: is a type of GO:0016747; is a type of catalytic activity, acting on a tRNA [GO:0140101] Sources: EC:2.3.1.234